{
  "term_id": "GO:0035529",
  "gene": "UniProtKB:P53370",
  "gene_name": "Nucleoside diphosphate-linked moiety X motif 6",
  "gene_symbol": "NUDT6",
  "term_label": "NADH pyrophosphatase activity"
}